{
  "gene_symbol": "CRTAP",
  "gene": "UniProtKB:O75718",
  "term_label": "collagen binding",
  "gene_name": "Cartilage-associated protein",
  "term_id": "GO:0005518"
}